potassium ion transmembrane transporter activity [GO:0015079] (molecular function) Sources: GOC:ai Relationships: is a type of metal ion transmembrane transporter activity [GO:0046873]; is part of GO:0071805 Definition: Enables the transfer of potassium ions (K+) from one side of a membrane to the other. Also known as: potassium transporter activity, potassium uptake permease activity, potassium uptake transmembrane transporter activity Subtypes: potassium channel activity [GO:0005267], GO:0008556, potassium:sodium symporter activity [GO:0009674], potassium:chloride symporter activity [GO:0015379], potassium:proton symporter activity [GO:0015387], amino acid:potassium symporter activity [GO:0017032], potassium ion uniporter activity [GO:0022819], solute:potassium antiporter activity [GO:0022821], high-affinity potassium ion transmembrane transporter activity [GO:0140107] Regulation: RO_0002212 by negative regulation of potassium ion transmembrane transporter activity [GO:1901017]